interleukin-30 production [GO:0072633] (biological process) Definition: The appearance of interleukin-30 due to biosynthesis or secretion following a cellular stimulus, resulting in an increase in its intracellular or extracellular levels. Also known as: IL-30 production, interleukin-30 complex production, interleukin-30 secretion References: PMID:30328794 Sources: GOC:BHF, GOC:mah Relationships: is a type of GO:0001816